pyrroloquinoline-quinone synthase activity [GO:0033732] (molecular function) Sources: EC:1.3.3.11, RHEA:10692 Definition: Catalysis of the reaction: 6-(2-amino-2-carboxyethyl)-7,8-dioxo-1,2,3,4,7,8-hexahydroquinoline-2,4-dicarboxylate + 3 O2 = 2 H2O + 2 H2O2 + H+ + pyrroloquinoline quinone. Also known as: 6-(2-amino-2-carboxyethyl)-7,8-dioxo-1,2,3,4,5,6,7,8-octahydroquinoline-2,4-dicarboxylate:oxygen oxidoreductase (cyclizing) activity, PqqC Relationships: is a type of oxidoreductase activity, acting on the CH-CH group of donors, oxygen as acceptor [GO:0016634]